{
  "gene_name": "KH domain-containing RNA-binding protein QKI",
  "gene": "UniProtKB:Q96PU8",
  "gene_symbol": "QKI",
  "term_id": "GO:0005634",
  "term_label": "nucleus"
}